{
  "term_id": "UNKNOWN:0003",
  "term_label": "Unknown cellular component",
  "gene_symbol": "CYP4F12",
  "gene_name": "Cytochrome P450 4F12",
  "gene": "UniProtKB:Q9HCS2"
}